leg disc anterior/posterior pattern formation [GO:0035200] (biological process) Definition: The establishment, maintenance and elaboration of the anterior/posterior axis of the leg imaginal disc. Sources: GOC:bf Relationships: is a type of anterior/posterior pattern specification, imaginal disc [GO:0007448]; is a type of leg disc pattern formation [GO:0035223]